{
  "gene": "UniProtKB:Q587J7",
  "term_id": "GO:0042078",
  "gene_symbol": "TDRD12",
  "term_label": "germ-line stem cell division",
  "gene_name": "Putative ATP-dependent RNA helicase TDRD12"
}